negative regulation of lysine biosynthetic process via alpha-aminoadipate and saccharopine [GO:2001195] (BP) Relationships: is a type of negative regulation of lysine biosynthetic process via aminoadipic acid [GO:1902987]; is_a GO:2001194; negatively regulates lysine biosynthetic process via alpha-aminoadipate and saccharopine [GO:0051975] Sources: GOC:obol Also known as: negative regulation of lysine biosynthesis via aminoadipic acid and saccharopine, negative regulation of lysine biosynthetic process via aminoadipic acid and saccharopine Definition: Any process that stops, prevents or reduces the frequency, rate or extent of lysine biosynthetic process via alpha-aminoadipate and saccharopine.